positive regulation of sexual sporulation resulting in formation of a cellular spore [GO:0043941] (biological process) Definition: Any process that activates, maintains or increases the frequency, rate or extent of the formation of cellular spores derived from the products of meiosis. Sources: GOC:pamgo_curators Relationships: is a type of regulation of sexual sporulation resulting in formation of a cellular spore [GO:0043940]; is a type of positive regulation of sporulation resulting in formation of a cellular spore [GO:0045881]; is a type of positive regulation of meiotic cell cycle [GO:0051446]; positively regulates GO:0043935 Subtypes: positive regulation of oospore formation [GO:0075245], positive regulation of ascospore formation [GO:0075296], GO:0075299, GO:0075303